{
  "term_label": "Unknown molecular function",
  "gene_symbol": "SIRPB1",
  "term_id": "UNKNOWN:0001",
  "gene": "UniProtKB:O00241",
  "gene_name": "Signal-regulatory protein beta-1"
}